{
  "gene": "UniProtKB:Q9NRY5",
  "gene_name": "Protein FAM114A2",
  "term_label": "Unknown biological process",
  "gene_symbol": "FAM114A2",
  "term_id": "UNKNOWN:0002"
}